1-aminocyclopropane-1-carboxylate biosynthetic process [GO:0042218] (biological process) Definition: The chemical reactions and pathways resulting in the formation of 1-aminocyclopropane-1-carboxylate, a natural product found in plant tissues. It is a key intermediate in the biosynthesis of ethylene (ethene), a fruit-ripening hormone in plants. Sources: GOC:go_curators Also known as: 1-aminocyclopropane-1-carboxylate anabolism, 1-aminocyclopropane-1-carboxylate biosynthesis, 1-aminocyclopropane-1-carboxylate formation, 1-aminocyclopropane-1-carboxylate synthesis Relationships: is a type of 1-aminocyclopropane-1-carboxylate metabolic process [GO:0018871]; is_a non-proteinogenic amino acid biosynthetic process [GO:0170043]; is a type of alpha-amino acid biosynthetic process [GO:1901607]